alpha-glucan biosynthetic process [GO:0030979] (biological process) Definition: The chemical reactions and pathways resulting in the formation of alpha-glucans, compounds composed of glucose residues linked by alpha-D-glucosidic bonds. Also known as: alpha-glucan anabolism, alpha-glucan biosynthesis, alpha-glucan formation, alpha-glucan synthesis Relationships: is a type of GO:0009250; is a type of GO:0030978 Regulation: regulated by regulation of alpha-glucan biosynthetic process [GO:0032949] Subtypes: reuteran biosynthetic process [GO:0052784], (1->3)-alpha-glucan biosynthetic process [GO:0070596], (1->4)-alpha-glucan biosynthetic process [GO:0070630] Sources: GOC:mah